cytosolic [4Fe-4S] assembly scaffold complex [GO:1904564] (cellular component) Relationships: is a type of ATPase complex [GO:1904949]; is a type of GO:1990229 Also known as: CIA scaffold complex, Nbp35-Cfd1 ATPase complex, cytosolic scaffold protein complex References: PMID:26195633, PMID:34660592 Sources: GOC:bhm, GOC:rb, GO_REF:0000088 Definition: A heterotetrameric complex with weak ATPase activity that is capable of scaffolding a 4Fe-4S (iron-sulfur) cluster. In yeast, the subunits are Nbp35 and Cfd1. In humans, the subunits are NUBP1 and NUBP2.